{
  "term_label": "neuronal cell body",
  "gene_symbol": "CIB1",
  "gene": "UniProtKB:Q99828",
  "gene_name": "Calcium and integrin-binding protein 1",
  "term_id": "GO:0043025"
}